bile-acid 7alpha-dehydratase activity [GO:0033988] (molecular function) Relationships: is a type of GO:0016836 Definition: Catalysis of the reaction: 7alpha,12alpha-dihydroxy-3-oxochol-4-en-24-oate = 12alpha-hydroxy-3-oxochola-4,6-dien-24-oate + H2O. References: PMID:26650892 Sources: RHEA:10436 Also known as: 7alpha,12alpha-dihydroxy-3-oxochol-4-enoate hydro-lyase (12alpha-hydroxy-3-oxochola-4,6-dienoate-forming) activity, 7alpha,12alpha-dihydroxy-3-oxochol-4-enoate hydro-lyase activity, BA7 alpha dehydratase activity